{
  "gene_symbol": "SYT14",
  "term_label": "Unknown cellular component",
  "gene": "UniProtKB:Q8NB59",
  "term_id": "UNKNOWN:0003",
  "gene_name": "Synaptotagmin-14"
}